cellular response to type I interferon [GO:0071357] (biological process) Definition: Any process that results in a change in state or activity of a cell (in terms of movement, secretion, enzyme production, gene expression, etc.) as a result of a type I interferon stimulus. Type I interferons include the interferon-alpha, beta, delta, episilon, zeta, kappa, tau, and omega gene families. Sources: GOC:mah Also known as: cellular response to type I IFN Relationships: is a type of response to type I interferon [GO:0034340]; is a type of cellular response to cytokine stimulus [GO:0071345]